{
  "gene_name": "Fc receptor-like protein 6",
  "gene_symbol": "FCRL6",
  "term_id": "GO:0006955",
  "gene": "UniProtKB:Q6DN72",
  "term_label": "immune response"
}